{
  "gene_symbol": "CFHR4",
  "gene": "UniProtKB:Q92496",
  "term_id": "GO:0006956",
  "gene_name": "Complement factor H-related protein 4",
  "term_label": "complement activation"
}